cyanide biosynthetic process [GO:0046202] (biological process) Sources: GOC:ai Definition: The chemical reactions and pathways resulting in the formation of cyanide, NC-, the anion of hydrocyanic acid. Cyanide is a potent inhibitor of respiration. Relationships: is a type of biosynthetic process [GO:0009058]; is_a cyanide metabolic process [GO:0019499] Also known as: cyanide anabolism, cyanide biosynthesis, cyanide formation, cyanide synthesis